{
  "gene_symbol": "MTMR3",
  "term_label": "phosphatidylinositol dephosphorylation",
  "term_id": "GO:0046856",
  "gene": "UniProtKB:Q13615",
  "gene_name": "Myotubularin-related protein 3"
}